{
  "gene_symbol": "LIFR",
  "term_id": "GO:0005127",
  "gene": "UniProtKB:P42702",
  "term_label": "ciliary neurotrophic factor receptor binding",
  "gene_name": "Leukemia inhibitory factor receptor"
}